{
  "gene_symbol": "ASGR1",
  "term_id": "GO:0038187",
  "gene": "UniProtKB:P07306",
  "gene_name": "Asialoglycoprotein receptor 1",
  "term_label": "pattern recognition receptor activity"
}